{
  "gene_symbol": "LTA",
  "term_id": "GO:0006955",
  "gene": "UniProtKB:P01374",
  "term_label": "immune response",
  "gene_name": "Lymphotoxin-alpha"
}